{
  "gene_symbol": "SLC22A16",
  "term_id": "UNKNOWN:0003",
  "gene_name": "Solute carrier family 22 member 16",
  "gene": "UniProtKB:Q86VW1",
  "term_label": "Unknown cellular component"
}